negative regulation of heart contraction [GO:0045822] (biological process) Sources: GOC:go_curators Subtypes: negative regulation of the force of heart contraction involved in baroreceptor response to increased systemic arterial blood pressure [GO:0001986], GO:0003108, negative regulation of heart rate [GO:0010459], negative regulation of cardiac muscle contraction [GO:0055118] Definition: Any process that stops, prevents, or reduces the frequency, rate or extent of heart contraction. Also known as: down regulation of heart contraction, down-regulation of heart contraction, downregulation of heart contraction, inhibition of heart contraction, negative regulation of cardiac contraction Relationships: is a type of GO:0008016; is_a negative regulation of blood circulation [GO:1903523]; negatively regulates heart contraction [GO:0060047]